{
  "term_id": "UNKNOWN:0002",
  "term_label": "Unknown biological process",
  "gene": "UniProtKB:Q5SRR4",
  "gene_name": "Lymphocyte antigen 6 complex locus protein G5c",
  "gene_symbol": "LY6G5C"
}